{
  "term_label": "immune response",
  "gene": "UniProtKB:A0A0C4DH25",
  "term_id": "GO:0006955",
  "gene_name": "Immunoglobulin kappa variable 3D-20",
  "gene_symbol": "IGKV3D-20"
}